{
  "term_id": "GO:0031012",
  "term_label": "extracellular matrix",
  "gene_name": "Fibulin-5",
  "gene": "UniProtKB:Q9UBX5",
  "gene_symbol": "FBLN5"
}